taxane 10-beta-hydroxylase activity [GO:0050597] (molecular function) Also known as: taxane 10b-hydroxylase activity, 5-alpha-taxadienol-10-beta-hydroxylase activity, taxa-4(20),11-dien-5alpha-yl acetate,NADPH:oxygen oxidoreductase (10beta-hydroxylating), taxane 10beta-hydroxylase activity Relationships: is a type of oxidoreductase activity, acting on paired donors, with incorporation or reduction of molecular oxygen, NAD(P)H as one donor, and incorporation of one atom of oxygen [GO:0016709] Sources: EC:1.14.14.105, RHEA:15241 Definition: Catalysis of the reaction: H+ + NADPH + O2 + taxa-4(20),11-dien-5alpha-yl acetate = 10beta-hydroxytaxa-4(20),11-dien-5alpha-yl acetate + H2O + NADP+.